{
  "term_id": "UNKNOWN:0003",
  "gene": "UniProtKB:Q6P6B7",
  "gene_name": "Ankyrin repeat domain-containing protein 16",
  "gene_symbol": "ANKRD16",
  "term_label": "Unknown cellular component"
}